4-hydroxybenzoate geranyltransferase activity [GO:0102930] (MF) Definition: Catalysis of the reaction: geranyl diphosphate + 4-hydroxybenzoic acid = 3-geranyl-4-hydroxybenzoate + diphosphoric acid. Sources: GOC:pz, RHEA:27854 Relationships: is_a transferase activity, transferring alkyl or aryl (other than methyl) groups [GO:0016765]